{
  "term_id": "GO:0005758",
  "term_label": "mitochondrial intermembrane space",
  "gene_name": "ADP-ribosylation factor-like protein 2-binding protein",
  "gene_symbol": "ARL2BP",
  "gene": "UniProtKB:Q9Y2Y0"
}